{
  "gene": "UniProtKB:Q9C010",
  "gene_symbol": "PKIB",
  "gene_name": "cAMP-dependent protein kinase inhibitor beta",
  "term_label": "Unknown biological process",
  "term_id": "UNKNOWN:0002"
}